{
  "gene_symbol": "MYOCOS",
  "gene_name": "Myocilin opposite strand protein",
  "gene": "UniProtKB:A0A1B0GUC4",
  "term_id": "UNKNOWN:0003",
  "term_label": "Unknown cellular component"
}